{
  "term_label": "cell adhesion",
  "gene": "UniProtKB:Q9BZA8",
  "term_id": "GO:0007155",
  "gene_name": "Protocadherin-11 Y-linked",
  "gene_symbol": "PCDH11Y"
}